repressor of RNA polymerase inhibitor activity [GO:0140871] (molecular function) Definition: Binds to and stops, prevents or reduces the activity of an RNA polymerase inhibitor. References: PMID:28475895, PMID:31048766 Relationships: is a type of molecular function inhibitor activity [GO:0140678]; negatively regulates RNA polymerase activity [GO:0097747]; negatively regulates GO:0140870